mating pheromone activity [GO:0000772] (molecular function) Relationships: is_a GO:0005186 Sources: GOC:clt, GOC:elh Definition: The activity of binding to and activating specific cell surface receptors, thereby inducing a behavioral or physiological response(s) from a responding organism or cell that leads to the transfer or union of genetic material between organisms or cells. The mating pheromone can either be retained on the cell surface or secreted.